{
  "gene_symbol": "BTC",
  "gene": "UniProtKB:P35070",
  "term_label": "positive regulation of cell population proliferation",
  "term_id": "GO:0008284",
  "gene_name": "Probetacellulin"
}